cerebellar granular layer development [GO:0021681] (biological process) Definition: The process whose specific outcome is the progression of the cerebellar granule layer over time, from its formation to the mature structure. The granular layer is the innermost layer of the cerebellar cortex. This layer contains densely packed small neurons, mostly granule cells. Some Golgi cells are found at the outer border. Granule neurons send parallel fibers to the upper molecular layer, where they synapse with Purkinje cell dendrites. Mossy fibers from the pontine nuclei in the white matter synapse with granule cell axons, Golgi cell axons and unipolar brush interneuron axons at cerebellar glomeruli in the granule cell layer. Sources: GOC:cls, GOC:dgh, GOC:dph, GOC:jid, GO_REF:0000021 Relationships: is a type of anatomical structure development [GO:0048856]; is part of cerebellar cortex development [GO:0021695]